{
  "gene_name": "NADP-dependent malic enzyme, mitochondrial",
  "term_label": "malate metabolic process",
  "gene": "UniProtKB:Q16798",
  "term_id": "GO:0006108",
  "gene_symbol": "ME3"
}